pilus organization [GO:0043711] (biological process) Also known as: pilus organisation, pilus organization and biogenesis Subtypes: GO:0009297, GO:0043108 Note: Note that this term should not be used for direct annotation. Please use one of the children, GO:0009297 ; pilus assembly or GO:0043108 ; pilus retraction. Relationships: is a type of cell projection organization [GO:0030030] Definition: A process that is carried out at the cellular level which results in the assembly, arrangement of constituent parts, or disassembly of a pilus, a short filamentous structure on a bacterial cell, flagella-like in structure and generally present in many copies. Sources: GOC:jl